{
  "term_id": "GO:0043473",
  "gene": "UniProtKB:Q969F9",
  "gene_symbol": "HPS3",
  "gene_name": "BLOC-2 complex member HPS3",
  "term_label": "pigmentation"
}